{
  "gene": "UniProtKB:Q8NHY6",
  "gene_symbol": "ZFP28",
  "gene_name": "Zinc finger protein 28 homolog",
  "term_id": "GO:0005634",
  "term_label": "nucleus"
}